positive regulation of synaptic metaplasticity [GO:0031918] (biological process) Definition: A process that increases synaptic metaplasticity. Metaplasticity is a higher-order form of plasticity and is manifest as a change in the ability to induce subsequent synaptic plasticity that is the ability of synapses to change as circumstances require. References: PMID:8658594 Sources: GOC:mah Also known as: up regulation of synaptic metaplasticity, up-regulation of synaptic metaplasticity, upregulation of synaptic metaplasticity, activation of synaptic metaplasticity, stimulation of synaptic metaplasticity Relationships: is a type of positive regulation of synaptic plasticity [GO:0031915]; is a type of regulation of synaptic metaplasticity [GO:0031916]